Tic complex [GO:0031897] (CC) Definition: The translocon of the inner envelope of chloroplasts, which facilitates the import of proteins across the chloroplast inner membrane. References: PMID:12180471, PMID:12393016 Also known as: chloroplast inner membrane translocase complex Relationships: is a type of membrane protein complex [GO:0098796]; is part of chloroplast inner membrane [GO:0009706]